{
  "gene": "UniProtKB:P51793",
  "gene_symbol": "CLCN4",
  "term_id": "GO:0005247",
  "gene_name": "H(+)_Cl(-) exchange transporter 4",
  "term_label": "voltage-gated chloride channel activity"
}